{
  "gene": "UniProtKB:Q2M3G4",
  "term_label": "cell morphogenesis",
  "gene_symbol": "SHROOM1",
  "gene_name": "Protein Shroom1",
  "term_id": "GO:0000902"
}